{
  "gene": "UniProtKB:Q68DD2",
  "term_label": "ruffle membrane",
  "gene_name": "Cytosolic phospholipase A2 zeta",
  "term_id": "GO:0032587",
  "gene_symbol": "PLA2G4F"
}